extracellular matrix organization in marginal zone involved in cerebral cortex radial glia guided migration [GO:0021820] (biological process) References: PMID:12626695 Sources: GOC:cls, GOC:dgh, GOC:dph, GOC:jid, GO_REF:0000021 Definition: The process that leads to the deposition of extracellular matrix signals in the marginal zone of the developing cerebral cortex. This extracellular matrix controls the movement of migrating cells. In mammals, the matrix is modified by Cajal-Retzius cells. Relationships: is a type of GO:0030198; is part of layer formation in cerebral cortex [GO:0021819] Also known as: extracellular matrix organisation in marginal zone involved in cerebral cortex radial glia guided migration, organization of extracellular matrix in the marginal zone involved in cerebral cortex glial-mediated radial migration